{
  "term_label": "phosphatase inhibitor activity",
  "gene_name": "Acidic leucine-rich nuclear phosphoprotein 32 family member E",
  "term_id": "GO:0019212",
  "gene_symbol": "ANP32E",
  "gene": "UniProtKB:Q9BTT0"
}